{
  "term_id": "UNKNOWN:0003",
  "gene": "UniProtKB:P0DPF4",
  "gene_name": "T cell receptor alpha variable 35",
  "gene_symbol": "TRAV35",
  "term_label": "Unknown cellular component"
}